{
  "term_id": "GO:0005615",
  "gene_name": "Otogelin-like protein",
  "term_label": "extracellular space",
  "gene_symbol": "OTOGL",
  "gene": "UniProtKB:Q3ZCN5"
}